{
  "term_id": "GO:0002682",
  "term_label": "regulation of immune system process",
  "gene": "UniProtKB:P24278",
  "gene_symbol": "ZBTB25",
  "gene_name": "Zinc finger and BTB domain-containing protein 25"
}